pollen tube reception [GO:0010483] (biological process) References: PMID:37640641 Definition: An interaction between the pollen tube, part of the male gametophyte, and the female gametophyte (typically the synergid cells), that results in the arrest of pollen tube growth, rupture of the pollen tube and the release of the sperm cells. Relationships: is a type of GO:0051703; is part of pollination [GO:0009856]